{
  "gene_name": "Eukaryotic translation initiation factor 2 subunit 2",
  "gene": "UniProtKB:P20042",
  "gene_symbol": "EIF2S2",
  "term_id": "GO:0031369",
  "term_label": "translation initiation factor binding"
}